{
  "gene_symbol": "RTP5",
  "gene": "UniProtKB:Q14D33",
  "term_id": "GO:0006612",
  "gene_name": "Receptor-transporting protein 5",
  "term_label": "protein targeting to membrane"
}